receptor ligand inhibitor activity [GO:0141069] (molecular function) References: PMID:12478285, PMID:1721860 Relationships: is a type of molecular function inhibitor activity [GO:0140678]; negatively regulates receptor ligand activity [GO:0048018] Definition: Binds to and decreases the activity of the ligand of a signaling receptor. Also known as: signaling receptor ligand inhibitor activity